regulation of colon smooth muscle contraction [GO:1904341] (BP) Definition: Any process that modulates the frequency, rate or extent of colon smooth muscle contraction. Relationships: is_a regulation of gastro-intestinal system smooth muscle contraction [GO:1904304]; regulates GO:1990765 References: PMID:24170253 Sources: GOC:TermGenie, GO_REF:0000058 Subtypes: negative regulation of colon smooth muscle contraction [GO:1904342], GO:1904343